{
  "term_id": "GO:0005125",
  "term_label": "cytokine activity",
  "gene": "UniProtKB:P01570",
  "gene_name": "Interferon alpha-14",
  "gene_symbol": "IFNA14"
}